{
  "term_id": "GO:0000712",
  "gene_name": "RecQ-mediated genome instability protein 1",
  "term_label": "resolution of meiotic recombination intermediates",
  "gene_symbol": "RMI1",
  "gene": "UniProtKB:Q9H9A7"
}